{
  "gene_symbol": "IRS4",
  "gene": "UniProtKB:O14654",
  "term_id": "GO:0005829",
  "gene_name": "Insulin receptor substrate 4",
  "term_label": "cytosol"
}